{
  "gene": "UniProtKB:P01566",
  "gene_name": "Interferon alpha-10",
  "term_id": "GO:0006959",
  "term_label": "humoral immune response",
  "gene_symbol": "IFNA10"
}